broad specificity oxidative DNA demethylase activity [GO:0035516] (molecular function) Note: This reaction directly reverses the alkylation on a nucleotide within DNA. Do not confuse with 5-methylcytosine dioxygenase activity ; GO:0070579, which removes the methyl group from position 5 of cytosine in DNA via oxidation of the 5-methylcytosine, followed by removal of the oxidated base by the base excision repair system. Also known as: oxidative DNA demethylase activity, 2-oxoglutarate-dependent DNA demethylase, 1-ethyladenine demethylase activity, 5-formylcytosine dioxygenase activity, 5-hydroxymethylcytosine dioxygenase activity, 5fC dioxygenase, 5hmC dioxygenase, N1-methyladenine demethylase activity, N3-methylcytosine demethylase activity References: PMID:12594517, PMID:16482161, PMID:18775698, PMID:19786499 Sources: RHEA:30299 Definition: Catalysis of the reaction: a methylated nucleobase within DNA + 2-oxoglutarate + O2 = a nucleobase within DNA + formaldehyde + succinate + CO2. Catalyzes oxidative demethylation of the DNA base lesions N1- methyladenine, N3-methylcytosine, N1-methylguanine, and N3- methylthymine. Can also act of RNA. Relationships: is a type of GO:0016706; is a type of DNA demethylase activity [GO:0035514]